negative regulation of intracellular signal transduction [GO:1902532] (biological process) Relationships: is a type of GO:0009968; is a type of regulation of intracellular signal transduction [GO:1902531]; negatively regulates intracellular signal transduction [GO:0035556] Also known as: down regulation of intracellular signal transduction, down regulation of intracellular signaling chain, down-regulation of intracellular signal transduction, down-regulation of intracellular signaling chain, downregulation of intracellular signal transduction, downregulation of intracellular signaling chain, negative regulation of intracellular protein kinase cascade, negative regulation of intracellular signaling cascade, negative regulation of intracellular signaling chain, down regulation of intracellular signal transduction pathway, down regulation of intracellular signaling cascade, down regulation of signal transmission via intracellular cascade, down-regulation of intracellular signal transduction pathway, downregulation of intracellular signal transduction pathway, downregulation of intracellular signaling cascade, downregulation of signal transmission via intracellular cascade, inhibition of intracellular signal transduction, inhibition of intracellular signal transduction pathway, inhibition of intracellular signaling cascade, inhibition of intracellular signaling chain, inhibition of signal transmission via intracellular cascade, negative regulation of intracellular signal transduction pathway, negative regulation of signal transmission via intracellular cascade, down regulation of intracellular signaling pathway, down regulation of signal transduction via intracellular signaling cascade, down-regulation of intracellular signaling cascade, down-regulation of intracellular signaling pathway, down-regulation of signal transduction via intracellular signaling cascade, down-regulation of signal transmission via intracellular cascade, downregulation of intracellular signaling pathway, downregulation of signal transduction via intracellular signaling cascade, inhibition of intracellular signaling pathway, inhibition of signal transduction via intracellular signaling cascade, negative regulation of intracellular signaling pathway, negative regulation of signal transduction via intracellular signaling cascade Sources: GOC:TermGenie, GOC:dph, GOC:signaling, GOC:tb Subtypes: negative regulation of thyroid hormone receptor signaling pathway [GO:0002156], negative regulation of nitric oxide mediated signal transduction [GO:0010751], GO:0032007, negative regulation of intracellular steroid hormone receptor signaling pathway [GO:0033144], negative regulation of hippo signaling [GO:0035331], negative regulation of peroxisome proliferator activated receptor signaling pathway [GO:0035359], negative regulation of cytoplasmic pattern recognition receptor signaling pathway [GO:0039532], GO:0043124, negative regulation of MAPK cascade [GO:0043409], negative regulation of retinoic acid receptor signaling pathway [GO:0048387], GO:0050849, negative regulation of small GTPase mediated signal transduction [GO:0051058], negative regulation of phosphatidylinositol 3-kinase/protein kinase B signal transduction [GO:0051898], negative regulation of SMAD protein signal transduction [GO:0060392], negative regulation of phosphorelay signal transduction system [GO:0070298], GO:0070303, negative regulation of vitamin D receptor signaling pathway [GO:0070563], negative regulation of protein kinase C signaling [GO:0090038], negative regulation of cAMP/PKA signal transduction [GO:0141162], negative regulation of phospholipase C/protein kinase C signal transduction [GO:0160195], negative regulation of endoplasmic reticulum unfolded protein response [GO:1900102], GO:1901223, negative regulation of signal transduction by p53 class mediator [GO:1901797], GO:1901977, negative regulation of hypoxia-inducible factor-1alpha signaling pathway [GO:1902072], negative regulation of SREBP signaling pathway [GO:2000639], negative regulation of intrinsic apoptotic signaling pathway [GO:2001243] Definition: Any process that stops, prevents or reduces the frequency, rate or extent of intracellular signal transduction.